{
  "gene_symbol": "CLIC3",
  "term_label": "chloride transport",
  "gene": "UniProtKB:O95833",
  "term_id": "GO:0006821",
  "gene_name": "Chloride intracellular channel protein 3"
}